{
  "gene": "UniProtKB:P15313",
  "gene_symbol": "ATP6V1B1",
  "term_id": "GO:0007035",
  "gene_name": "V-type proton ATPase subunit B, kidney isoform",
  "term_label": "vacuolar acidification"
}